mesonephric S-shaped body morphogenesis [GO:0061244] (biological process) Relationships: is a type of S-shaped body morphogenesis [GO:0072050]; is part of mesonephric nephron morphogenesis [GO:0061228] Definition: The process in which the mesonephric S-shaped body is generated and organized. The mesonephric S-shaped body is the successor of the mesonephric comma-shaped body that contributes to the morphogenesis of a nephron in the mesonephros. Sources: GOC:mtg_kidney_jan10